positive regulation of encysted zoospore germination [GO:0075228] (biological process) Definition: Any process that activates, maintains or increases the frequency, rate or extent of encysted zoospore germination. Also known as: positive regulation of encysted zoospore germination on or near host Relationships: is a type of regulation of encysted zoospore germination [GO:0075227]; is a type of positive regulation of spore germination [GO:1904361]; positively regulates encysted zoospore germination [GO:0075226] Sources: GOC:pamgo_curators